{
  "gene_symbol": "DPH3P1",
  "term_label": "iron ion binding",
  "gene_name": "Putative DPH3 homolog B",
  "term_id": "GO:0005506",
  "gene": "UniProtKB:Q9H4G8"
}